{
  "gene_symbol": "TENT5C",
  "term_label": "poly(A) RNA polymerase activity",
  "term_id": "GO:1990817",
  "gene_name": "Terminal nucleotidyltransferase 5C",
  "gene": "UniProtKB:Q5VWP2"
}